{
  "term_label": "Unknown molecular function",
  "gene": "UniProtKB:Q9BRN9",
  "gene_name": "TM2 domain-containing protein 3",
  "term_id": "UNKNOWN:0001",
  "gene_symbol": "TM2D3"
}